{
  "term_label": "Unknown cellular component",
  "gene": "UniProtKB:Q8IYL3",
  "gene_symbol": "C1orf174",
  "term_id": "UNKNOWN:0003",
  "gene_name": "UPF0688 protein C1orf174"
}